{
  "gene_name": "Glycosylphosphatidylinositol anchor attachment 1 protein",
  "term_id": "GO:0016255",
  "gene": "UniProtKB:O43292",
  "gene_symbol": "GPAA1",
  "term_label": "attachment of GPI anchor to protein"
}